{
  "gene": "UniProtKB:Q3KRA9",
  "gene_symbol": "ALKBH6",
  "gene_name": "Alpha-ketoglutarate-dependent dioxygenase alkB homolog 6",
  "term_label": "Unknown biological process",
  "term_id": "UNKNOWN:0002"
}